{
  "gene": "UniProtKB:Q5U649",
  "term_label": "Unknown cellular component",
  "gene_symbol": "C12orf60",
  "gene_name": "Uncharacterized protein C12orf60",
  "term_id": "UNKNOWN:0003"
}